{
  "term_label": "regulation of DNA-templated transcription",
  "term_id": "GO:0006355",
  "gene_symbol": "ZNF735",
  "gene_name": "Putative zinc finger protein 735",
  "gene": "UniProtKB:P0CB33"
}